F-9775B catabolic process [GO:1900613] (biological process) Also known as: F-9775B breakdown, F-9775B catabolism, F-9775B degradation Sources: GOC:TermGenie, GOC:di Relationships: is a type of phenol-containing compound catabolic process [GO:0019336]; is_a polyketide catabolic process [GO:0030640] Definition: The chemical reactions and pathways resulting in the breakdown of F-9775B.